{
  "gene_symbol": "SCOC",
  "term_id": "GO:0005802",
  "term_label": "trans-Golgi network",
  "gene_name": "Short coiled-coil protein",
  "gene": "UniProtKB:Q9UIL1"
}